{
  "gene": "UniProtKB:Q14626",
  "gene_symbol": "IL11RA",
  "gene_name": "Interleukin-11 receptor subunit alpha",
  "term_label": "external side of plasma membrane",
  "term_id": "GO:0009897"
}